regulation of intestinal absorption [GO:1904478] (biological process) Subtypes: regulation of intestinal D-glucose absorption [GO:1903985], negative regulation of intestinal absorption [GO:1904479], positive regulation of intestinal absorption [GO:1904480], regulation of intestinal lipid absorption [GO:1904729] References: PMID:12469120 Sources: GOC:BHF, GOC:TermGenie, GOC:rl, GO_REF:0000058 Relationships: is a type of regulation of digestive system process [GO:0044058]; regulates intestinal absorption [GO:0050892] Definition: Any process that modulates the frequency, rate or extent of intestinal absorption.